{
  "term_id": "GO:0005829",
  "gene": "UniProtKB:O14744",
  "gene_name": "Protein arginine N-methyltransferase 5",
  "gene_symbol": "PRMT5",
  "term_label": "cytosol"
}